maintenance of protein complex location [GO:0098544] (biological process) Sources: GOC:dos Definition: Any process in which a protein complex is maintained in a location and prevented from moving elsewhere. These include sequestration, stabilization to prevent transport elsewhere and the active retrieval of protein complexes that move away. Subtypes: maintenance of protein complex location in cytoplasm [GO:0098545] Relationships: is a type of GO:0051235